postsynaptic specialization membrane of symmetric synapse [GO:0099164] (cellular component) Relationships: is a type of postsynaptic specialization membrane [GO:0099634]; is part of postsynaptic specialization of symmetric synapse [GO:0099629] Sources: GOC:dos Definition: The membrane component of the postsynaptic specialization of a symmetric synapse. This is the region of the postsynaptic membrane in which the population of neurotransmitter receptors involved in synaptic transmission are concentrated.